{
  "term_id": "GO:0008083",
  "gene": "UniProtKB:P21741",
  "gene_name": "Midkine",
  "term_label": "growth factor activity",
  "gene_symbol": "MDK"
}